{
  "term_id": "UNKNOWN:0003",
  "gene_name": "WD repeat- and FYVE domain-containing protein 4",
  "term_label": "Unknown cellular component",
  "gene": "UniProtKB:Q6ZS81",
  "gene_symbol": "WDFY4"
}